{
  "gene_symbol": "MSANTD5",
  "term_id": "UNKNOWN:0003",
  "term_label": "Unknown cellular component",
  "gene": "UniProtKB:A0A3B3IT52",
  "gene_name": "Putative uncharacterized protein MSANTD5"
}